chemokine (C-C motif) ligand 12 binding [GO:0035716] (molecular function) Sources: GOC:BHF Also known as: CCL12 binding Definition: Binding to chemokine (C-C motif) ligand 12. Relationships: is a type of C-C chemokine binding [GO:0019957]